regulation of phytol biosynthetic process [GO:1904963] (biological process) References: PMID:24275650 Sources: GOC:TermGenie, GO_REF:0000058 Definition: Any process that modulates the frequency, rate or extent of phytol biosynthetic process. Subtypes: positive regulation of phytol biosynthetic process [GO:1904964] Also known as: regulation of phytol anabolism, regulation of phytol biosynthesis, regulation of phytol formation, regulation of phytol synthesis Relationships: is a type of regulation of isoprenoid metabolic process [GO:0019747]; is a type of GO:0046890; is a type of regulation of alcohol biosynthetic process [GO:1902930]; regulates phytol biosynthetic process [GO:0033520]